{
  "gene_name": "Dedicator of cytokinesis protein 4",
  "term_id": "GO:0005085",
  "gene_symbol": "DOCK4",
  "gene": "UniProtKB:Q8N1I0",
  "term_label": "guanyl-nucleotide exchange factor activity"
}